cell-cell junction assembly [GO:0007043] (biological process) Also known as: intercellular junction assembly Definition: The aggregation, arrangement and bonding together of a set of components to form a junction between cells. Relationships: is a type of GO:0034329; is a type of cell-cell junction organization [GO:0045216] Subtypes: desmosome assembly [GO:0002159], gap junction assembly [GO:0016264], paranodal junction assembly [GO:0030913], adherens junction assembly [GO:0034333], filtration diaphragm assembly [GO:0036058], apical junction assembly [GO:0043297], tight junction assembly [GO:0120192] Sources: GOC:ai